response to exogenous dsRNA [GO:0043330] (biological process) Sources: GOC:go_curators Subtypes: GO:0071360 Relationships: is a type of response to dsRNA [GO:0043331] Definition: Any process that results in a change in state or activity of a cell or an organism (in terms of movement, secretion, enzyme production, gene expression, etc.) as a result of an exogenous double-stranded RNA stimulus. Also known as: response to exogenous double-stranded RNA, response to viral dsRNA Note: Note that the presence of exogenous double-stranded RNA is usually indicative of a viral infection. Consider also annotating to 'response to virus ; GO:0009615'.